{
  "gene_name": "Zinc finger protein 250",
  "gene_symbol": "ZNF250",
  "gene": "UniProtKB:P15622",
  "term_id": "GO:0000981",
  "term_label": "DNA-binding transcription factor activity, RNA polymerase II-specific"
}